hypusine metabolic process [GO:0046516] (biological process) Also known as: hypusine metabolism Sources: GOC:ai Relationships: is a type of modified amino acid metabolic process [GO:0006575]; is a type of L-amino acid metabolic process [GO:0170033]; is a type of non-proteinogenic amino acid metabolic process [GO:0170041] Definition: The chemical reactions and pathways involving hypusine, N6-(4-amino-2-hydroxybutyl)-L-lysine.